{
  "gene_symbol": "MOGAT2",
  "term_id": "GO:0006651",
  "gene_name": "2-acylglycerol O-acyltransferase 2",
  "gene": "UniProtKB:Q3SYC2",
  "term_label": "diacylglycerol biosynthetic process"
}